{
  "gene": "UniProtKB:Q96S55",
  "term_label": "single-stranded DNA helicase activity",
  "term_id": "GO:0017116",
  "gene_symbol": "WRNIP1",
  "gene_name": "ATPase WRNIP1"
}